{
  "term_id": "UNKNOWN:0001",
  "term_label": "Unknown molecular function",
  "gene": "UniProtKB:Q12794",
  "gene_symbol": "HYAL1",
  "gene_name": "Hyaluronidase-1"
}